{
  "gene_symbol": "KRT28",
  "gene": "UniProtKB:Q7Z3Y7",
  "term_id": "GO:0045095",
  "gene_name": "Keratin, type I cytoskeletal 28",
  "term_label": "keratin filament"
}